{
  "gene_name": "DENN domain-containing protein 2C",
  "gene_symbol": "DENND2C",
  "gene": "UniProtKB:Q68D51",
  "term_label": "Unknown biological process",
  "term_id": "UNKNOWN:0002"
}